{
  "gene": "UniProtKB:Q8N2I9",
  "term_label": "Unknown cellular component",
  "gene_name": "Serine_threonine-protein kinase 40",
  "term_id": "UNKNOWN:0003",
  "gene_symbol": "STK40"
}